regulation of steroid hormone secretion [GO:2000831] (biological process) Relationships: is a type of regulation of lipid transport [GO:0032368]; is a type of regulation of endocrine process [GO:0044060]; is a type of regulation of hormone secretion [GO:0046883]; regulates steroid hormone secretion [GO:0035929] Sources: GOC:sl Subtypes: regulation of ecdysteroid secretion [GO:0007555], negative regulation of steroid hormone secretion [GO:2000832], GO:2000833, regulation of androgen secretion [GO:2000834], regulation of corticosteroid hormone secretion [GO:2000846], GO:2000861, regulation of estradiol secretion [GO:2000864], regulation of estrone secretion [GO:2000867], regulation of progesterone secretion [GO:2000870] Definition: Any process that modulates the frequency, rate or extent of steroid hormone secretion.